response to vitamin B1 [GO:0010266] (biological process) Definition: Any process that results in a change in state or activity of a cell or an organism (in terms of movement, secretion, enzyme production, gene expression, etc.) as a result of a vitamin B1 stimulus. Sources: GOC:pz Also known as: response to thiamin, response to thiamine Relationships: is a type of response to vitamin [GO:0033273]; is a type of GO:0097305; is a type of response to nitrogen compound [GO:1901698] Subtypes: cellular response to vitamin B1 [GO:0071301]